{
  "gene_symbol": "PARG",
  "term_label": "poly(ADP-ribose) glycohydrolase activity",
  "gene_name": "Poly(ADP-ribose) glycohydrolase",
  "term_id": "GO:0004649",
  "gene": "UniProtKB:Q86W56"
}